{
  "gene_name": "Semenogelin-1",
  "gene": "UniProtKB:P04279",
  "term_id": "UNKNOWN:0001",
  "term_label": "Unknown molecular function",
  "gene_symbol": "SEMG1"
}